betaine-homocysteine S-methyltransferase activity [GO:0047150] (molecular function) Sources: EC:2.1.1.5, RHEA:22336 Also known as: betaine-homocysteine methyltransferase activity, betaine-homocysteine transmethylase activity, trimethylammonioacetate:L-homocysteine S-methyltransferase activity Relationships: is a type of S-methyltransferase activity [GO:0008172] Definition: Catalysis of the reaction: L-homocysteine + glycine betaine = N,N-dimethylglycine + L-methionine.